{
  "gene_symbol": "SCN1B",
  "term_label": "membrane depolarization during cardiac muscle cell action potential",
  "gene": "UniProtKB:Q07699",
  "term_id": "GO:0086012",
  "gene_name": "Sodium channel subunit beta-1"
}